{
  "gene": "UniProtKB:Q9BSB4",
  "gene_name": "Autophagy-related protein 101",
  "term_id": "GO:0019901",
  "gene_symbol": "ATG101",
  "term_label": "protein kinase binding"
}